{
  "term_label": "calcium-dependent cysteine-type endopeptidase activity",
  "gene_symbol": "CAPN1",
  "term_id": "GO:0004198",
  "gene": "UniProtKB:P07384",
  "gene_name": "Calpain-1 catalytic subunit"
}